positive regulation of hemostasis [GO:1900048] (biological process) Relationships: is_a GO:0048518; is a type of regulation of hemostasis [GO:1900046]; RO_0002213 hemostasis [GO:0007599] Subtypes: positive regulation of blood coagulation [GO:0030194] Sources: GOC:TermGenie Definition: Any process that activates or increases the frequency, rate or extent of hemostasis. Also known as: up regulation of hemostasis, up-regulation of hemostasis, upregulation of hemostasis, activation of hemostasis